{
  "gene_name": "Monoacylglycerol lipase ABHD2",
  "term_id": "GO:0051793",
  "gene": "UniProtKB:P08910",
  "gene_symbol": "ABHD2",
  "term_label": "medium-chain fatty acid catabolic process"
}